{
  "term_label": "Unknown biological process",
  "term_id": "UNKNOWN:0002",
  "gene_symbol": "GAL3ST4",
  "gene": "UniProtKB:Q96RP7",
  "gene_name": "Galactose-3-O-sulfotransferase 4"
}